UDP-N-acetylglucosamine 1-carboxyvinyltransferase activity [GO:0008760] (MF) Relationships: is a type of GO:0016765 Definition: Catalysis of the reaction: phosphoenolpyruvate + UDP-N-acetyl-alpha-D-glucosamine = phosphate + UDP-N-acetyl-3-O-(1-carboxyvinyl)-D-glucosamine. Sources: EC:2.5.1.7, RHEA:18681 Also known as: MurA transferase activity, UDP-N-acetylglucosamine 1-carboxyvinyl-transferase activity, UDP-N-acetylglucosamine enoylpyruvyltransferase activity, enoylpyruvate transferase activity, phosphoenolpyruvate-UDP-acetylglucosamine-3-enolpyruvyltransferase activity, phosphoenolpyruvate:UDP-2-acetamido-2-deoxy-D-glucose 2-enoyl-1-carboxyethyltransferase activity, phosphoenolpyruvate:UDP-N-acetyl-D-glucosamine 1-carboxyvinyltransferase activity, phosphoenolpyruvate:uridine diphosphate N-acetylglucosamine enolpyruvyltransferase activity, phosphoenolpyruvate:uridine-5'-diphospho-N-acetyl-2-amino-2-deoxyglucose 3-enolpyruvyltransferase activity, phosphopyruvate-uridine diphosphoacetylglucosamine pyruvatetransferase activity, pyruvate-UDP-acetylglucosamine transferase activity, pyruvate-uridine diphospho-N-acetyl-glucosamine transferase activity, pyruvate-uridine diphospho-N-acetylglucosamine transferase activity, pyruvic-uridine diphospho-N-acetylglucosaminyltransferase activity